{
  "gene_symbol": "SAMD10",
  "gene_name": "Sterile alpha motif domain-containing protein 10",
  "gene": "UniProtKB:Q9BYL1",
  "term_label": "cytoplasmic side of plasma membrane",
  "term_id": "GO:0009898"
}